{
  "gene_name": "Ubiquitin carboxyl-terminal hydrolase isozyme L5",
  "term_id": "GO:0004843",
  "gene": "UniProtKB:Q9Y5K5",
  "gene_symbol": "UCHL5",
  "term_label": "cysteine-type deubiquitinase activity"
}